{
  "gene": "UniProtKB:Q9UBS0",
  "gene_symbol": "RPS6KB2",
  "term_label": "cytoplasm",
  "gene_name": "Ribosomal protein S6 kinase beta-2",
  "term_id": "GO:0005737"
}